left ventral flagellum [GO:0097558] (cellular component) References: PMID:16607022, PMID:5961344 Sources: GOC:giardia, ISBN:9780124260207 Also known as: left ventral cilium Definition: A cilium (also called flagellum) found in Giardia species (trophozoite stage). It is nucleated by the left ventral basal body and exits the cell body proximally and dorsal to the ventral disc. Relationships: is a type of GO:0097729 Note: Note that we deem cilium and microtubule-based flagellum to be equivalent; the primary term name reflects frequency of use. Also note that, due to the asymmetric nature of the Giardia trophozoite, this term is defined spatially as the trophozoite is viewed from the dorsal side, with the two nuclei dorsal to the ventral disc, and the ventral disc toward the anterior.